{
  "gene_symbol": "CASC3",
  "term_id": "GO:0035145",
  "gene": "UniProtKB:O15234",
  "term_label": "exon-exon junction complex",
  "gene_name": "Protein CASC3"
}